{
  "term_id": "GO:0071013",
  "term_label": "catalytic step 2 spliceosome",
  "gene_symbol": "SF3B2",
  "gene": "UniProtKB:Q13435",
  "gene_name": "Splicing factor 3B subunit 2"
}